{
  "gene_symbol": "ITGB3",
  "term_label": "fibrinogen binding",
  "term_id": "GO:0070051",
  "gene": "UniProtKB:P05106",
  "gene_name": "Integrin beta-3"
}